{
  "term_label": "cytoplasm",
  "gene": "UniProtKB:P98082",
  "gene_name": "Disabled homolog 2",
  "gene_symbol": "DAB2",
  "term_id": "GO:0005737"
}